{
  "gene": "UniProtKB:P09486",
  "gene_symbol": "SPARC",
  "term_id": "GO:0031012",
  "gene_name": "SPARC",
  "term_label": "extracellular matrix"
}